benzoate catabolic process via hydroxylation [GO:0043640] (biological process) Also known as: benzoate breakdown via hydroxylation, benzoate degradation via hydroxylation Sources: GOC:jl, MetaCyc:PWY-2503 Definition: The chemical reactions and pathways resulting in the breakdown of benzoate, by its hydroxylation to cis-1,2-dihydroxybenzoate followed by dehydrogenation to catechol. Relationships: is a type of benzoate catabolic process [GO:0043639]